{
  "gene": "UniProtKB:Q9NZI5",
  "gene_symbol": "GRHL1",
  "gene_name": "Grainyhead-like protein 1 homolog",
  "term_id": "GO:0006357",
  "term_label": "regulation of transcription by RNA polymerase II"
}